{
  "gene_symbol": "CLDN3",
  "term_label": "cell-cell adhesion mediator activity",
  "term_id": "GO:0098632",
  "gene": "UniProtKB:O15551",
  "gene_name": "Claudin-3"
}